{
  "gene_name": "Glutamate receptor ionotropic, kainate 2",
  "gene_symbol": "GRIK2",
  "term_id": "GO:0042734",
  "term_label": "presynaptic membrane",
  "gene": "UniProtKB:Q13002"
}